{
  "gene_name": "Putative protocadherin beta-18",
  "gene_symbol": "PCDHB18P",
  "term_label": "plasma membrane",
  "gene": "UniProtKB:Q96TA0",
  "term_id": "GO:0005886"
}